{
  "term_id": "UNKNOWN:0002",
  "gene": "UniProtKB:A6NGS2",
  "gene_name": "Glutamate-rich protein 4",
  "term_label": "Unknown biological process",
  "gene_symbol": "ERICH4"
}